{
  "gene_symbol": "FCHSD1",
  "term_id": "UNKNOWN:0001",
  "gene": "UniProtKB:Q86WN1",
  "term_label": "Unknown molecular function",
  "gene_name": "F-BAR and double SH3 domains protein 1"
}